{
  "term_id": "GO:1990446",
  "term_label": "U1 snRNP binding",
  "gene": "UniProtKB:Q86U06",
  "gene_name": "Probable RNA-binding protein 23",
  "gene_symbol": "RBM23"
}